{
  "term_label": "endosome organization",
  "gene": "UniProtKB:Q2M389",
  "gene_symbol": "WASHC4",
  "term_id": "GO:0007032",
  "gene_name": "WASH complex subunit 4"
}